{
  "gene": "UniProtKB:Q9H633",
  "gene_symbol": "RPP21",
  "gene_name": "Ribonuclease P protein subunit p21",
  "term_label": "Unknown molecular function",
  "term_id": "UNKNOWN:0001"
}